{
  "gene_symbol": "CIMAP1B",
  "term_label": "Unknown biological process",
  "gene": "UniProtKB:A8MYP8",
  "term_id": "UNKNOWN:0002",
  "gene_name": "Outer dense fiber protein 3B"
}